{
  "term_id": "UNKNOWN:0002",
  "gene_symbol": "PALD1",
  "gene_name": "Paladin",
  "gene": "UniProtKB:Q9ULE6",
  "term_label": "Unknown biological process"
}